{
  "gene": "UniProtKB:Q8IYT8",
  "term_id": "GO:0048675",
  "term_label": "axon extension",
  "gene_symbol": "ULK2",
  "gene_name": "Serine_threonine-protein kinase ULK2"
}